trimethylamine receptor activity [GO:1990081] (molecular function) Relationships: is a type of trace-amine receptor activity [GO:0001594] Definition: Combining with the biogenic amine trimethylamine to initiate a change in cell activity. References: PMID:16878137